{
  "term_label": "nucleus",
  "gene_name": "Transcriptional adapter 2-alpha",
  "gene_symbol": "TADA2A",
  "gene": "UniProtKB:O75478",
  "term_id": "GO:0005634"
}